{
  "term_id": "GO:0005886",
  "gene_symbol": "PIP4P2",
  "gene_name": "Type 2 phosphatidylinositol 4,5-bisphosphate 4-phosphatase",
  "term_label": "plasma membrane",
  "gene": "UniProtKB:Q8N4L2"
}